cellulase activity [GO:0008810] (molecular function) Also known as: beta-1,4-endoglucan hydrolase activity, beta-1,4-glucanase activity, endo-1,4-beta-D-glucanase activity, endo-1,4-beta-D-glucanohydrolase activity, endo-1,4-beta-glucanase activity, endoglucanase activity, alkali cellulase activity, carboxymethyl cellulase activity, 1,4-(1,3;1,4)-beta-D-glucan 4-glucanohydrolase activity, 9.5 cellulase activity, avicelase activity, celluase A, celludextrinase activity, cellulase A 3, cellulosin AP, endoglucanase D, pancellase SS Sources: EC:3.2.1.4 Definition: Catalysis of the endohydrolysis of (1->4)-beta-D-glucosidic linkages in cellulose, lichenin and cereal beta-D-glucans. Relationships: is_a GO:0004553